{
  "gene_symbol": "PDE6B",
  "gene_name": "Rod cGMP-specific 3',5'-cyclic phosphodiesterase subunit beta",
  "gene": "UniProtKB:P35913",
  "term_label": "3',5'-cyclic-GMP phosphodiesterase activity",
  "term_id": "GO:0047555"
}